facial suture morphogenesis [GO:0097096] (biological process) Sources: GOC:pr, GOC:sl, Wikipedia:Cranial_sutures, Wikipedia:Head_and_neck_anatomy#Musculoskeletal_system Definition: The process in which any suture between facial bones is generated and organized. Subtypes: nasal suture morphogenesis [GO:0097097] Relationships: is a type of craniofacial suture morphogenesis [GO:0097094]